{
  "gene": "UniProtKB:A6NGW2",
  "term_id": "GO:0009986",
  "term_label": "cell surface",
  "gene_name": "Putative stereocilin-like protein",
  "gene_symbol": "STRCP1"
}